{
  "term_label": "Unknown molecular function",
  "gene": "UniProtKB:O15172",
  "term_id": "UNKNOWN:0001",
  "gene_symbol": "PSPHP1",
  "gene_name": "Putative phosphoserine phosphatase-like protein"
}